leucoplast organization [GO:0009659] (biological process) Sources: GOC:jid Also known as: leucoplast organisation, leucoplast organization and biogenesis Relationships: is a type of plastid organization [GO:0009657] Subtypes: elaioplast organization [GO:0043579] Definition: A process that is carried out at the cellular level which results in the assembly, arrangement of constituent parts, or disassembly of a leucoplast. A leucoplast is a colorless plastid involved in the synthesis of monoterpenes.